{
  "term_label": "plasma membrane",
  "gene_symbol": "LRRC32",
  "gene_name": "Transforming growth factor beta activator LRRC32",
  "gene": "UniProtKB:Q14392",
  "term_id": "GO:0005886"
}